dendritic spine development [GO:0060996] (biological process) Relationships: is a type of anatomical structure development [GO:0048856]; is part of dendrite development [GO:0016358] Definition: The process whose specific outcome is the progression of the dendritic spine over time, from its formation to the mature structure. A dendritic spine is a protrusion from a dendrite and a specialized subcellular compartment involved in synaptic transmission. Regulation: regulated by GO:0060998; positively regulated by positive regulation of dendritic spine development [GO:0060999]; negatively regulated by GO:0061000 Sources: GOC:dph